{
  "gene_symbol": "RAB9B",
  "gene": "UniProtKB:Q9NP90",
  "term_id": "GO:0005770",
  "gene_name": "Ras-related protein Rab-9B",
  "term_label": "late endosome"
}